{
  "term_id": "GO:0000398",
  "gene": "UniProtKB:O75400",
  "gene_name": "Pre-mRNA-processing factor 40 homolog A",
  "term_label": "mRNA splicing, via spliceosome",
  "gene_symbol": "PRPF40A"
}